{
  "term_label": "GTPase activator activity",
  "gene": "UniProtKB:O14559",
  "term_id": "GO:0005096",
  "gene_name": "Rho GTPase-activating protein 33",
  "gene_symbol": "ARHGAP33"
}